{
  "gene_name": "E3 ubiquitin-protein ligase CBL-C",
  "gene": "UniProtKB:Q9ULV8",
  "term_label": "negative regulation of epidermal growth factor receptor signaling pathway",
  "gene_symbol": "CBLC",
  "term_id": "GO:0042059"
}